{
  "gene": "UniProtKB:P30533",
  "gene_name": "Alpha-2-macroglobulin receptor-associated protein",
  "term_id": "GO:0005793",
  "term_label": "endoplasmic reticulum-Golgi intermediate compartment",
  "gene_symbol": "LRPAP1"
}